{
  "term_label": "Unknown molecular function",
  "gene_symbol": "GFOD1",
  "gene_name": "Glucose-fructose oxidoreductase domain-containing protein 1",
  "gene": "UniProtKB:Q9NXC2",
  "term_id": "UNKNOWN:0001"
}